{
  "gene_symbol": "ST13",
  "gene": "UniProtKB:P50502",
  "term_label": "Unknown cellular component",
  "term_id": "UNKNOWN:0003",
  "gene_name": "Hsc70-interacting protein"
}